{
  "term_id": "GO:0097401",
  "term_label": "synaptic vesicle lumen acidification",
  "gene": "UniProtKB:O95670",
  "gene_symbol": "ATP6V1G2",
  "gene_name": "V-type proton ATPase subunit G 2"
}